{
  "gene_name": "IQ motif and SEC7 domain-containing protein 2",
  "gene": "UniProtKB:Q5JU85",
  "term_id": "GO:0005085",
  "gene_symbol": "IQSEC2",
  "term_label": "guanyl-nucleotide exchange factor activity"
}